{
  "gene": "UniProtKB:Q9NSE2",
  "term_label": "negative regulation of receptor signaling pathway via JAK-STAT",
  "gene_name": "Cytokine-inducible SH2-containing protein",
  "gene_symbol": "CISH",
  "term_id": "GO:0046426"
}